{
  "term_id": "GO:0006508",
  "gene_symbol": "PLG",
  "term_label": "proteolysis",
  "gene_name": "Plasminogen",
  "gene": "UniProtKB:P00747"
}